{
  "gene": "UniProtKB:Q9UMS0",
  "gene_name": "NFU1 iron-sulfur cluster scaffold homolog, mitochondrial",
  "term_id": "GO:0051539",
  "gene_symbol": "NFU1",
  "term_label": "4 iron, 4 sulfur cluster binding"
}